early phagosome lumen [GO:0062113] (cellular component) Also known as: early phagocytic vesicle lumen Relationships: is a type of GO:0097013; is part of GO:0032009 References: PMID:18813294 Definition: The volume enclosed by the membrane of an early phagosome.